{
  "gene": "UniProtKB:Q1W4C9",
  "gene_name": "Serine protease inhibitor Kazal-type 13",
  "term_id": "UNKNOWN:0003",
  "term_label": "Unknown cellular component",
  "gene_symbol": "SPINK13"
}